positive regulation of error-prone translesion synthesis [GO:1904333] (biological process) Definition: Any process that activates or increases the frequency, rate or extent of error-prone translesion synthesis. References: PMID:22761594 Sources: GOC:TermGenie, GOC:kmv, GO_REF:0000058 Also known as: positive regulation of mutagenic PRR, up regulation of error-prone translesion synthesis, up regulation of mutagenic PRR, up-regulation of error-prone translesion synthesis, up-regulation of mutagenic PRR, upregulation of error-prone translesion synthesis, upregulation of mutagenic PRR, activation of error-prone translesion synthesis, activation of mutagenic PRR, activation of error-prone postreplication DNA repair, activation of mutagenic postreplication DNA repair, positive regulation of error-prone postreplication DNA repair, positive regulation of mutagenic postreplication DNA repair, up regulation of error-prone postreplication DNA repair, up regulation of mutagenic postreplication DNA repair, up-regulation of error-prone postreplication DNA repair, up-regulation of mutagenic postreplication DNA repair, upregulation of error-prone postreplication DNA repair, upregulation of mutagenic postreplication DNA repair Relationships: is a type of positive regulation of response to stimulus [GO:0048584]; is a type of regulation of error-prone translesion synthesis [GO:1904331]; is a type of GO:2000573; positively regulates error-prone translesion synthesis [GO:0042276]